created by [oboInOwl#created:by]